{
  "gene_symbol": "SERPINI1",
  "gene_name": "Neuroserpin",
  "gene": "UniProtKB:Q99574",
  "term_id": "GO:0004867",
  "term_label": "serine-type endopeptidase inhibitor activity"
}